{
  "gene_name": "Aprataxin",
  "gene": "UniProtKB:Q7Z2E3",
  "term_label": "nucleus",
  "term_id": "GO:0005634",
  "gene_symbol": "APTX"
}